histone H4K deacetylase activity [GO:0141051] (molecular function) Definition: Removal of an acetyl group from a lysine residue in a histone H4. Relationships: is a type of histone deacetylase activity [GO:0004407] Note: Histone deacytylase (HDAC) enzymes are divided into four classes: the Class I Rpd3-like proteins (in human: HDAC1, HDAC2, HDAC3, and HDAC8); the Class II Hda1-like proteins (in human: HDAC4, HDAC5, HDAC6, HDAC7, HDAC9, and HDAC10); the Class III Sir2-like proteins (in human: SIRT1, SIRT2, SIRT3, SIRT4, SIRT5, SIRT6, and SIRT7); and the Class IV protein (HDAC11 in human). Except for Class III enzymes, the mechanism is a metal-dependent hydrolysis of the acetylated substrate. The Class III HDACs use NAD+ as a reactant to deacetylate acetyl lysine residues of protein substrates forming nicotinamide, the deacetylated product, and the metabolite 2'-O-acetyl-ADP-ribose. Therefore, Class III are classified as transferases (EC:2) and others are hydrolases (EC:3). Subtypes: histone H4K16 deacetylase activity, hydrolytic mechanism [GO:0034739], histone H4K16 deacetylase activity, NAD-dependent [GO:0046970], GO:0140937, GO:0180032, histone H4K8 deacetylase activity, hydrolytic mechanism [GO:0180033] References: PMID:12590135